{
  "term_id": "GO:0030674",
  "gene": "UniProtKB:Q7Z4S9",
  "gene_symbol": "SH2D6",
  "term_label": "protein-macromolecule adaptor activity",
  "gene_name": "SH2 domain-containing protein 6"
}